SAS acetyltransferase complex [GO:0033255] (CC) Definition: A protein complex that possesses histone acetyltransferase activity and links histone acetylation to the assembly of transcriptionally silent chromatin. In vitro, the complex acetylates lysine 16 of histone H4 and lysine 14 of histone H3, although the latter may not be relevant in vivo. The complex contains a catalytic subunit and at least two other subunits; in Saccharomyces, the catalytic subunit is Sas2p and additional subunits are Sas4p and Sas5p. Relationships: is a type of piccolo histone acetyltransferase complex [GO:0032777] Also known as: SAS-I complex References: PMID:11731480, PMID:12626510, PMID:15788653